{
  "gene_symbol": "FREM2",
  "gene": "UniProtKB:Q5SZK8",
  "term_label": "extracellular matrix",
  "gene_name": "FRAS1-related extracellular matrix protein 2",
  "term_id": "GO:0031012"
}